negative regulation of smooth muscle contraction involved in micturition [GO:1904319] (biological process) Relationships: is a type of negative regulation of smooth muscle contraction [GO:0045986]; is_a regulation of smooth muscle contraction involved in micturition [GO:1904318]; negatively regulates smooth muscle contraction involved in micturition [GO:0060083] Definition: Any process that stops, prevents or reduces the frequency, rate or extent of smooth muscle contraction involved in micturition. References: PMID:18562635 Sources: GOC:TermGenie, GO_REF:0000058 Also known as: down regulation of smooth muscle contraction involved in micturition, down-regulation of smooth muscle contraction involved in micturition, downregulation of smooth muscle contraction involved in micturition, inhibition of smooth muscle contraction involved in micturition, down regulation of smooth muscle contraction involved in urination, down regulation of urinary bladder smooth muscle contraction involved in micturition, down-regulation of smooth muscle contraction involved in urination, down-regulation of urinary bladder smooth muscle contraction involved in micturition, downregulation of smooth muscle contraction involved in urination, downregulation of urinary bladder smooth muscle contraction involved in micturition, inhibition of smooth muscle contraction involved in urination, inhibition of urinary bladder smooth muscle contraction involved in micturition, negative regulation of smooth muscle contraction involved in urination, negative regulation of urinary bladder smooth muscle contraction involved in micturition